{
  "gene_name": "Angiopoietin-1 receptor",
  "gene": "UniProtKB:Q02763",
  "gene_symbol": "TEK",
  "term_label": "positive regulation of endothelial cell migration",
  "term_id": "GO:0010595"
}